{
  "gene_symbol": "ZNF552",
  "gene_name": "Zinc finger protein 552",
  "term_id": "GO:0006357",
  "term_label": "regulation of transcription by RNA polymerase II",
  "gene": "UniProtKB:Q9H707"
}